{
  "gene_symbol": "FAM237A",
  "gene_name": "Protein FAM237A",
  "term_id": "UNKNOWN:0001",
  "gene": "UniProtKB:A0A1B0GTK4",
  "term_label": "Unknown molecular function"
}